{
  "term_id": "GO:0001708",
  "gene_symbol": "TBX20",
  "gene": "UniProtKB:Q9UMR3",
  "term_label": "cell fate specification",
  "gene_name": "T-box transcription factor TBX20"
}